aminoglycoside 3''-adenylyltransferase activity [GO:0009012] (molecular function) Relationships: is a type of aminoglycoside nucleotidyltransferase activity [GO:0034068] Sources: EC:2.7.7.47, RHEA:20245 Definition: Catalysis of the reaction: ATP + streptomycin = 3''-adenylylstreptomycin + diphosphate + H+. Also known as: ATP:streptomycin 3''-adenylyltransferase activity, streptomycin 3''-adenylyltransferase activity, AAD (3'')